{
  "gene": "UniProtKB:Q99848",
  "gene_symbol": "EBNA1BP2",
  "term_id": "UNKNOWN:0001",
  "term_label": "Unknown molecular function",
  "gene_name": "Probable rRNA-processing protein EBP2"
}